cell periphery [GO:0071944] (cellular component) Definition: The broad region around and including the plasma membrane of a cell, encompassing the cell cortex (inside the cell), the plasma membrane, and any external encapsulating structures. Relationships: is a type of cellular anatomical structure [GO:0110165] Sources: GOC:pdt